{
  "term_label": "Unknown molecular function",
  "gene_symbol": "BLOC1S3",
  "gene": "UniProtKB:Q6QNY0",
  "term_id": "UNKNOWN:0001",
  "gene_name": "Biogenesis of lysosome-related organelles complex 1 subunit 3"
}